{
  "term_label": "T cell costimulation",
  "gene": "UniProtKB:Q9Y6W8",
  "gene_name": "Inducible T-cell costimulator",
  "gene_symbol": "ICOS",
  "term_id": "GO:0031295"
}